{
  "gene": "UniProtKB:O75908",
  "term_id": "GO:0005789",
  "gene_symbol": "SOAT2",
  "gene_name": "Sterol O-acyltransferase 2",
  "term_label": "endoplasmic reticulum membrane"
}